{
  "gene_symbol": "DCUN1D4",
  "term_label": "ubiquitin-like protein binding",
  "gene_name": "DCN1-like protein 4",
  "gene": "UniProtKB:Q92564",
  "term_id": "GO:0032182"
}